H zone [GO:0031673] (cellular component) Sources: GOC:mtg_muscle, ISBN:0321204131 Relationships: is_a cellular anatomical structure [GO:0110165]; is part of A band [GO:0031672] Definition: A relatively pale zone traversing the center of the A band of a sarcomere, visible in relaxed muscle fibers; consists of the central portion of thick (myosin) filaments that are not overlapped by thin (actin) filaments. Also known as: H band, H disc